anammoxosome [GO:0044222] (CC) Relationships: is a type of GO:0043231; is part of cytoplasm [GO:0005737] Definition: An intracytoplasmic membrane-bounded compartment in anaerobic ammonium oxidation (anammox) bacteria, is the site of anammox catabolism. References: PMID:17993524, PMID:19682260 Sources: GOC:dh